{
  "gene": "UniProtKB:P15735",
  "gene_name": "Phosphorylase b kinase gamma catalytic chain, liver_testis isoform",
  "term_id": "GO:0005737",
  "gene_symbol": "PHKG2",
  "term_label": "cytoplasm"
}